{
  "gene_symbol": "UGT1A5",
  "term_label": "liver development",
  "gene_name": "UDP-glucuronosyltransferase 1A5",
  "term_id": "GO:0001889",
  "gene": "UniProtKB:P35504"
}